{
  "term_label": "negative regulation of Wnt signaling pathway",
  "gene_symbol": "SOST",
  "gene_name": "Sclerostin",
  "gene": "UniProtKB:Q9BQB4",
  "term_id": "GO:0030178"
}